{
  "gene_symbol": "LILRB1",
  "term_id": "GO:0002767",
  "gene": "UniProtKB:Q8NHL6",
  "term_label": "immune response-inhibiting cell surface receptor signaling pathway",
  "gene_name": "Leukocyte immunoglobulin-like receptor subfamily B member 1"
}